ventral cochlear nucleus development [GO:0021749] (BP) Definition: The process whose specific outcome is the progression of the ventral cochlear nucleus over time, from its formation to the mature structure. Relationships: is a type of cochlear nucleus development [GO:0021747] Sources: GOC:cls, GOC:curators, GOC:dgh, GOC:dph, GOC:jid